{
  "term_label": "double-strand break repair via homologous recombination",
  "term_id": "GO:0000724",
  "gene_symbol": "RECQL5",
  "gene": "UniProtKB:O94762",
  "gene_name": "ATP-dependent DNA helicase Q5"
}